{
  "term_id": "GO:0043484",
  "gene_symbol": "RBM38",
  "gene": "UniProtKB:Q9H0Z9",
  "gene_name": "RNA-binding protein 38",
  "term_label": "regulation of RNA splicing"
}